{
  "gene": "UniProtKB:Q8WWG9",
  "term_label": "regulation of ventricular cardiac muscle cell membrane repolarization",
  "term_id": "GO:0060307",
  "gene_name": "Potassium voltage-gated channel subfamily E member 4",
  "gene_symbol": "KCNE4"
}